regulation of metanephric ureteric bud development [GO:2001074] (biological process) Relationships: is a type of regulation of metanephros development [GO:0072215]; regulates metanephric part of ureteric bud development [GO:0035502] Sources: GOC:obol Definition: Any process that modulates the frequency, rate or extent of metanephric ureteric bud development. Subtypes: negative regulation of metanephric ureteric bud development [GO:2001075], GO:2001076